{
  "gene": "UniProtKB:P28062",
  "term_id": "GO:0019774",
  "gene_name": "Proteasome subunit beta type-8",
  "gene_symbol": "PSMB8",
  "term_label": "proteasome core complex, beta-subunit complex"
}